{
  "term_label": "nodal signaling pathway",
  "gene": "UniProtKB:P0CG36",
  "gene_symbol": "CFC1B",
  "term_id": "GO:0038092",
  "gene_name": "Cryptic family protein 1B"
}